{
  "term_id": "GO:0015986",
  "term_label": "proton motive force-driven ATP synthesis",
  "gene": "UniProtKB:P36542",
  "gene_symbol": "ATP5F1C",
  "gene_name": "ATP synthase subunit gamma, mitochondrial"
}